negative regulation of dendrite development [GO:2000171] (biological process) Relationships: is a type of negative regulation of neuron projection development [GO:0010977]; is_a regulation of dendrite development [GO:0050773]; is a type of negative regulation of developmental process [GO:0051093]; negatively regulates dendrite development [GO:0016358] Sources: GOC:obol Definition: Any process that stops, prevents, or reduces the frequency, rate or extent of dendrite development.